glucosamine N-acetyltransferase activity [GO:0047932] (molecular function) Relationships: is a type of GO:0008080 Sources: EC:2.3.1.3, RHEA:21332 Also known as: acetyl-CoA:D-glucosamine N-acetyltransferase activity, glucosamine acetylase activity, glucosamine acetyltransferase activity Definition: Catalysis of the reaction: D-glucosamine + acetyl-CoA = N-acetyl-D-glucosamine + CoA + H+.